chlorophenol O-methyltransferase activity [GO:0030790] (molecular function) Definition: Catalysis of the reaction: S-adenosyl-L-methionine + trichlorophenol = S-adenosyl-L-homocysteine + trichloroanisole. Relationships: is a type of S-adenosylmethionine-dependent methyltransferase activity [GO:0008757] Sources: EC:2.1.1.136 Also known as: halogenated phenol O-methyltransferase activity, S-adenosyl-L-methionine:trichlorophenol O-methyltransferase activity, trichlorophenol O-methyltransferase activity